{
  "term_label": "integrin binding",
  "gene_name": "Integrin beta-1-binding protein 1",
  "gene": "UniProtKB:O14713",
  "gene_symbol": "ITGB1BP1",
  "term_id": "GO:0005178"
}